dTDP metabolic process [GO:0046072] (biological process) Definition: The chemical reactions and pathways involving dTDP, deoxyribosylthymine diphosphate. Subtypes: dTDP biosynthetic process [GO:0006233], dTDP catabolic process [GO:0006246] Sources: GOC:go_curators Relationships: is a type of GO:0009196; is a type of GO:0009219 Also known as: dTDP metabolism